low-affinity L-arginine transmembrane transporter activity [GO:0097626] (molecular function) Definition: Enables the transfer of L-arginine from one side of a membrane to the other. In low-affinity transport the transporter is able to bind the solute only if it is present at very high concentrations. References: PMID:8195186 Sources: GOC:krc Also known as: low affinity L-arginine transmembrane transporter activity Relationships: is a type of L-arginine transmembrane transporter activity [GO:0061459]; is a type of low-affinity basic amino acid transmembrane transporter activity [GO:0097625]